{
  "gene_symbol": "SLAMF6",
  "gene_name": "SLAM family member 6",
  "term_id": "GO:0006955",
  "term_label": "immune response",
  "gene": "UniProtKB:Q96DU3"
}